{
  "gene_name": "Proteasome subunit beta type-10",
  "term_label": "endopeptidase activity",
  "gene": "UniProtKB:P40306",
  "gene_symbol": "PSMB10",
  "term_id": "GO:0004175"
}